{
  "term_label": "RNA polymerase II cis-regulatory region sequence-specific DNA binding",
  "gene_symbol": "SP7",
  "gene_name": "Transcription factor Sp7",
  "term_id": "GO:0000978",
  "gene": "UniProtKB:Q8TDD2"
}